{
  "gene": "UniProtKB:Q9HCI5",
  "gene_symbol": "MAGEE1",
  "term_id": "GO:0005634",
  "term_label": "nucleus",
  "gene_name": "Melanoma-associated antigen E1"
}